L-proline transmembrane transporter activity [GO:0015193] (molecular function) Also known as: L-proline transporter activity, glycine betaine/proline porter activity, proline/glycine/betaine:hydrogen/sodium symporter activity, L-proline permease activity Definition: Enables the transfer of L-proline from one side of a membrane to the other. L-proline is pyrrolidine-2-carboxylic acid. Relationships: is a type of neutral L-amino acid transmembrane transporter activity [GO:0015175]; is a type of GO:0015179; is part of proline transmembrane transport [GO:0035524] Sources: GOC:ai, GOC:mtg_transport, ISBN:0815340729